{
  "gene_name": "Transcription intermediary factor 1-beta",
  "term_label": "chromatin binding",
  "gene": "UniProtKB:Q13263",
  "gene_symbol": "TRIM28",
  "term_id": "GO:0003682"
}